icosahedral viral capsid, neck [GO:0098030] (cellular component) Definition: A region of constriction located below the head and above the tail sheath of viruses with contractile tails (Myoviridae). Sources: GOC:bm Relationships: is_a virion component [GO:0044423]; is part of icosahedral viral capsid [GO:0019030]